{
  "gene": "UniProtKB:P58181",
  "gene_symbol": "OR10A3",
  "term_label": "olfactory receptor activity",
  "term_id": "GO:0004984",
  "gene_name": "Olfactory receptor 10A3"
}